{
  "gene_symbol": "CHCHD2P9",
  "term_id": "GO:0043565",
  "gene_name": "Putative coiled-coil-helix-coiled-coil-helix domain-containing protein CHCHD2P9, mitochondrial",
  "term_label": "sequence-specific DNA binding",
  "gene": "UniProtKB:Q5T1J5"
}